{
  "gene_name": "Protein GR6",
  "term_label": "Unknown biological process",
  "gene_symbol": "LINC01565",
  "gene": "UniProtKB:O15544",
  "term_id": "UNKNOWN:0002"
}